{
  "gene_symbol": "SERINC2",
  "gene_name": "Serine incorporator 2",
  "gene": "UniProtKB:Q96SA4",
  "term_label": "Unknown molecular function",
  "term_id": "UNKNOWN:0001"
}